cellular response to iron ion [GO:0071281] (biological process) Also known as: cellular response to iron Relationships: is a type of response to iron ion [GO:0010039]; is a type of GO:0071248 Sources: GOC:mah Definition: Any process that results in a change in state or activity of a cell (in terms of movement, secretion, enzyme production, gene expression, etc.) as a result of an iron ion stimulus. Subtypes: cellular response to iron(II) ion [GO:0071282], GO:0071283